positive regulation of metaphase/anaphase transition of meiosis I [GO:1905188] (biological process) Definition: Any process that activates or increases the frequency, rate or extent of metaphase/anaphase transition of meiosis I. Also known as: positive regulation of meiosis I metaphase/anaphase transition References: PMID:21389117 Sources: GOC:TermGenie, GO_REF:0000058 Relationships: is a type of GO:1902104; is a type of regulation of metaphase/anaphase transition of meiosis I [GO:1905186]; positively regulates metaphase/anaphase transition of meiosis I [GO:1990949]